{
  "term_label": "toll-like receptor 4 signaling pathway",
  "gene": "UniProtKB:P51617",
  "term_id": "GO:0034142",
  "gene_symbol": "IRAK1",
  "gene_name": "Interleukin-1 receptor-associated kinase 1"
}